{
  "term_label": "nucleolus",
  "gene_symbol": "WDR74",
  "term_id": "GO:0005730",
  "gene_name": "WD repeat-containing protein 74",
  "gene": "UniProtKB:Q6RFH5"
}